enterobactin binding [GO:1903981] (molecular function) Definition: Binding to enterobactin. Relationships: is a type of macrolide binding [GO:0005527]; is_a GO:0043168; is a type of heterocyclic compound binding [GO:1901363] References: PMID:21951132 Sources: GOC:TermGenie, GOC:mr, GO_REF:0000067 Also known as: siderophore binding, enterochelin binding